{
  "gene_symbol": "SLX9",
  "term_id": "UNKNOWN:0001",
  "gene": "UniProtKB:Q9NSI2",
  "gene_name": "Ribosome biogenesis protein SLX9 homolog",
  "term_label": "Unknown molecular function"
}